{
  "term_label": "Unknown cellular component",
  "term_id": "UNKNOWN:0003",
  "gene_name": "Coiled-coil domain-containing protein 74B",
  "gene": "UniProtKB:Q96LY2",
  "gene_symbol": "CCDC74B"
}